{
  "term_label": "sodium ion transmembrane transport",
  "gene": "UniProtKB:Q9Y5Y9",
  "gene_symbol": "SCN10A",
  "term_id": "GO:0035725",
  "gene_name": "Sodium channel protein type 10 subunit alpha"
}